{
  "gene": "UniProtKB:Q12852",
  "gene_name": "Mitogen-activated protein kinase kinase kinase 12",
  "term_id": "GO:0005737",
  "term_label": "cytoplasm",
  "gene_symbol": "MAP3K12"
}